{
  "gene_symbol": "NDOR1",
  "gene": "UniProtKB:Q9UHB4",
  "term_label": "cytosol",
  "gene_name": "NADPH-dependent diflavin oxidoreductase 1",
  "term_id": "GO:0005829"
}